{
  "term_label": "Unknown molecular function",
  "gene_name": "Ankyrin repeat domain-containing protein 61",
  "gene_symbol": "ANKRD61",
  "gene": "UniProtKB:A6NGH8",
  "term_id": "UNKNOWN:0001"
}